regulation of cell fate commitment [GO:0010453] (biological process) Relationships: is a type of regulation of developmental process [GO:0050793]; is a type of regulation of cellular process [GO:0050794]; regulates GO:0045165 Subtypes: negative regulation of cell fate commitment [GO:0010454], GO:0010455, regulation of cell fate specification [GO:0042659], regulation of retinal cone cell fate commitment [GO:0060222], GO:0060224, regulation of R7 cell fate commitment [GO:0106396], regulation of T-helper 17 cell lineage commitment [GO:2000328], regulation of venous endothelial cell fate commitment [GO:2000787] Sources: GOC:dph, GOC:tb Definition: Any process that modulates the frequency, rate or extent of cell fate commitment. Cell fate commitment is the commitment of cells to specific cell fates and their capacity to differentiate into particular kinds of cells. Positional information is established through protein signals that emanate from a localized source within a cell (the initial one-cell zygote) or within a developmental field.